{
  "term_label": "cardiac muscle contraction",
  "gene_name": "Myosin light chain 4",
  "gene_symbol": "MYL4",
  "gene": "UniProtKB:P12829",
  "term_id": "GO:0060048"
}